{
  "gene": "UniProtKB:A6NE52",
  "term_id": "UNKNOWN:0002",
  "gene_name": "WD repeat-containing protein 97",
  "gene_symbol": "WDR97",
  "term_label": "Unknown biological process"
}